{
  "gene_symbol": "LINC00477",
  "term_label": "Unknown cellular component",
  "gene": "UniProtKB:Q96M19",
  "gene_name": "Putative transmembrane protein encoded by LINC00477",
  "term_id": "UNKNOWN:0003"
}